{
  "term_id": "GO:0005615",
  "gene_name": "Transthyretin",
  "term_label": "extracellular space",
  "gene": "UniProtKB:P02766",
  "gene_symbol": "TTR"
}